{
  "gene": "UniProtKB:Q9P126",
  "gene_name": "C-type lectin domain family 1 member B",
  "term_id": "GO:0007165",
  "term_label": "signal transduction",
  "gene_symbol": "CLEC1B"
}